negative regulation of axon extension involved in regeneration [GO:0048692] (biological process) Relationships: is a type of GO:0030517; is a type of GO:0048688; is a type of GO:0048690; negatively regulates axon extension involved in regeneration [GO:0048677] Sources: GOC:dgh, GOC:dph, GOC:jid, GOC:lm Definition: Any process that stops, prevents, or reduces the frequency, rate or extent of axon extension involved in regeneration. Also known as: down regulation of axon extension involved in regeneration, down-regulation of axon extension involved in regeneration, downregulation of axon extension involved in regeneration, inhibition of axon extension involved in regeneration